termination of RNA polymerase II transcription, poly(A)-coupled [GO:0030846] (biological process) Definition: An RNA polymerase II transcription termination process in which cleavage and polyadenylylation of the mRNA 3' end are coupled to transcription termination. References: PMID:12944462, PMID:18679429, PMID:27371117 Sources: GOC:txnOH Also known as: termination of RNA polymerase II transcription, polyadenylation-coupled, transcription termination from Pol II promoter, RNA polymerase(A) coupled, transcription termination from Pol II promoter, poly(A) coupled Relationships: is a type of termination of RNA polymerase II transcription [GO:0006369] Regulation: regulated by regulation of termination of RNA polymerase II transcription, poly(A)-coupled [GO:2000804]; negatively regulated by negative regulation of termination of RNA polymerase II transcription, poly(A)-coupled [GO:2000805]; positively regulated by GO:2000806